{
  "gene_symbol": "GRIPAP1",
  "gene_name": "GRIP1-associated protein 1",
  "term_id": "GO:0099158",
  "gene": "UniProtKB:Q4V328",
  "term_label": "regulation of recycling endosome localization within postsynapse"
}